{
  "gene": "UniProtKB:Q9BY43",
  "term_id": "UNKNOWN:0001",
  "term_label": "Unknown molecular function",
  "gene_symbol": "CHMP4A",
  "gene_name": "Charged multivesicular body protein 4a"
}